{
  "term_label": "septin complex",
  "gene_name": "Septin-9",
  "gene": "UniProtKB:Q9UHD8",
  "term_id": "GO:0031105",
  "gene_symbol": "SEPTIN9"
}